{
  "term_id": "GO:0032456",
  "gene_name": "Ras-related protein Rab-13",
  "gene_symbol": "RAB13",
  "term_label": "endocytic recycling",
  "gene": "UniProtKB:P51153"
}